mitochondrial rRNA export from mitochondrion [GO:0019090] (biological process) Also known as: export of mitochondrial rRNA, mitochondrial rRNA export, mitochondrial rRNA export from mitochondria, mitochondrial rRNA export out of mitochondrion, mitochondrial rRNA transport from mitochondrion, mitochondrial rRNA, mitochondrial export Subtypes: GO:0019091, mitochondrial srRNA export from mitochondrion [GO:0019092] References: PMID:28115039 Sources: GOC:ai Relationships: is a type of GO:0051029; is a type of export from the mitochondrion [GO:0170037] Definition: The process in which a rRNA, ribosomal ribonucleic acid, is transported from the mitochondrial matrix into the cytosol.